{
  "gene": "UniProtKB:Q8IXP5",
  "gene_name": "POU domain class 2-associating factor 2",
  "term_id": "GO:0003713",
  "gene_symbol": "POU2AF2",
  "term_label": "transcription coactivator activity"
}